regulation of pectin biosynthetic process [GO:1900030] (biological process) Also known as: regulation of pectin anabolism, regulation of pectin biosynthesis, regulation of pectin formation, regulation of pectin synthesis Definition: Any process that modulates the frequency, rate or extent of pectin biosynthetic process. Relationships: is a type of regulation of polysaccharide biosynthetic process [GO:0032885]; regulates pectin biosynthetic process [GO:0045489] Sources: GOC:TermGenie